{
  "gene_symbol": "CPXM2",
  "term_id": "UNKNOWN:0002",
  "term_label": "Unknown biological process",
  "gene_name": "Inactive carboxypeptidase-like protein X2",
  "gene": "UniProtKB:Q8N436"
}